{
  "term_label": "endoplasmic reticulum to Golgi vesicle-mediated transport",
  "gene_symbol": "CTAGE9",
  "gene": "UniProtKB:A4FU28",
  "gene_name": "cTAGE family member 9",
  "term_id": "GO:0006888"
}